{
  "term_id": "GO:0031965",
  "term_label": "nuclear membrane",
  "gene_name": "Trimeric intracellular cation channel type A",
  "gene": "UniProtKB:Q9H6F2",
  "gene_symbol": "TMEM38A"
}